{
  "gene": "UniProtKB:P40939",
  "term_label": "long-chain (3S)-3-hydroxyacyl-CoA dehydrogenase (NAD+) activity",
  "term_id": "GO:0016509",
  "gene_name": "Trifunctional enzyme subunit alpha, mitochondrial",
  "gene_symbol": "HADHA"
}